{
  "term_label": "Unknown molecular function",
  "gene_symbol": "TRBV7-1",
  "term_id": "UNKNOWN:0001",
  "gene_name": "Probable non-functional T cell receptor beta variable 7-1",
  "gene": "UniProtKB:A0A0A6YYK4"
}